{
  "gene_symbol": "SLC22A14",
  "term_id": "UNKNOWN:0001",
  "term_label": "Unknown molecular function",
  "gene": "UniProtKB:Q9Y267",
  "gene_name": "Solute carrier family 22 member 14"
}